{
  "term_label": "lysosomal membrane",
  "gene_symbol": "CLN5",
  "gene_name": "Ceroid-lipofuscinosis neuronal protein 5",
  "gene": "UniProtKB:O75503",
  "term_id": "GO:0005765"
}